{
  "term_id": "GO:0006357",
  "gene_name": "Ligand-dependent nuclear receptor corepressor-like protein",
  "gene_symbol": "LCORL",
  "term_label": "regulation of transcription by RNA polymerase II",
  "gene": "UniProtKB:Q8N3X6"
}